{
  "term_label": "N-acetylglucosamine-6-sulfatase activity",
  "gene": "UniProtKB:P15586",
  "term_id": "GO:0008449",
  "gene_name": "N-acetylglucosamine-6-sulfatase",
  "gene_symbol": "GNS"
}